positive regulation of cell migration by vascular endothelial growth factor signaling pathway [GO:0038089] (biological process) Also known as: VEGF-induced cell migration, positive regulation of cell migration by VEGF signaling pathway, positive regulation of cell migration by vascular endothelial growth factor signalling pathway, VEGF-A-induced cell migration Sources: GOC:bf, GOC:signaling Definition: The series of molecular signals initiated by vascular endothelial growth factor (VEGF) binding to its receptor on the surface of a cell, which activates or increases the frequency, rate or extent of the orderly movement of a cell from one site to another. Subtypes: positive regulation of endothelial cell chemotaxis by VEGF-activated vascular endothelial growth factor receptor signaling pathway [GO:0038033], positive regulation of cell migration by VEGF-activated platelet derived growth factor receptor signaling pathway [GO:0038090] Relationships: is a type of positive regulation of cell migration [GO:0030335]; is a type of GO:0038084